glutathione synthase activity [GO:0004363] (molecular function) Sources: EC:6.3.2.3, RHEA:13557 Definition: Catalysis of the reaction: L-gamma-glutamyl-L-cysteine + ATP + glycine = ADP + glutathione + 2 H+ + phosphate. Relationships: is a type of acid-amino acid ligase activity [GO:0016881]; is a type of non-ribosomal peptide synthetase activity [GO:1904091]; is part of GO:0006750 Also known as: GSH synthetase activity, gamma-L-glutamyl-L-cysteine:glycine ligase (ADP-forming), glutathione synthetase activity